early endosome lumen [GO:0031905] (CC) Sources: GOC:mah Relationships: is a type of GO:0031904; is part of early endosome [GO:0005769] Definition: The volume enclosed by the membrane of an early endosome.